{
  "gene_symbol": "PRKD2",
  "term_label": "protein serine/threonine kinase activity",
  "term_id": "GO:0004674",
  "gene": "UniProtKB:Q9BZL6",
  "gene_name": "Serine_threonine-protein kinase D2"
}